{
  "term_label": "Unknown cellular component",
  "gene": "UniProtKB:P0C7T8",
  "gene_symbol": "TMEM253",
  "term_id": "UNKNOWN:0003",
  "gene_name": "Transmembrane protein 253"
}